{
  "term_label": "nucleus",
  "gene": "UniProtKB:Q96EP1",
  "term_id": "GO:0005634",
  "gene_name": "E3 ubiquitin-protein ligase CHFR",
  "gene_symbol": "CHFR"
}